{
  "gene": "UniProtKB:Q9H158",
  "term_id": "GO:0007155",
  "gene_symbol": "PCDHAC1",
  "gene_name": "Protocadherin alpha-C1",
  "term_label": "cell adhesion"
}